enterochelin esterase activity [GO:0008849] (molecular function) Also known as: enterobactin esterase activity Definition: Catalysis of the reaction: enterobactin + 3 H2O = 3 N-23-dihydroxybenzoyl-L-serine + 3 H+. References: PMID:4565531 Sources: MetaCyc:RXN0-1661 Relationships: is a type of hydrolase activity, acting on ester bonds [GO:0016788]